{
  "term_id": "GO:0005829",
  "gene_symbol": "DVL1P1",
  "term_label": "cytosol",
  "gene_name": "Putative segment polarity protein dishevelled homolog DVL1P1",
  "gene": "UniProtKB:P54792"
}